{
  "term_label": "cysteine biosynthetic process via cystathionine",
  "gene_name": "Cystathionine gamma-lyase",
  "gene": "UniProtKB:P32929",
  "term_id": "GO:0019343",
  "gene_symbol": "CTH"
}